monocyte activation involved in immune response [GO:0002280] (biological process) Also known as: monocyte activation during immune response References: PMID:16551245 Sources: GOC:add, ISBN:0781735149 Definition: The change in morphology and behavior of a monocyte resulting from exposure to a cytokine, chemokine, cellular ligand, or soluble factor, leading to the initiation or perpetuation of an immune response. Relationships: is a type of myeloid cell activation involved in immune response [GO:0002275]; is_a monocyte activation [GO:0042117]